{
  "gene_symbol": "XAGE3",
  "gene": "UniProtKB:Q8WTP9",
  "gene_name": "X antigen family member 3",
  "term_label": "Unknown cellular component",
  "term_id": "UNKNOWN:0003"
}